{
  "gene_name": "Plasminogen activator inhibitor 1",
  "term_id": "GO:0010757",
  "term_label": "negative regulation of plasminogen activation",
  "gene_symbol": "SERPINE1",
  "gene": "UniProtKB:P05121"
}